inositol-1,4,5,6-tetrakisphosphate 3-kinase activity [GO:0000824] (molecular function) Relationships: is a type of inositol tetrakisphosphate kinase activity [GO:0051765] Definition: Catalysis of the reaction: 1D-myo-inositol 1,4,5,6-tetrakisphosphate + ATP = 1D-myo-inositol 1,3,4,5,6-pentakisphosphate + ADP + H+. Also known as: 1D-myo-inositol-tetrakisphosphate 3-kinase activity, IpmK, inositol polyphosphate multikinase activity, inositol tetrakisphosphate 3-kinase activity, inositol 1,4,5,6-tetrakisphosphate 3-kinase activity Sources: RHEA:11856